{
  "term_label": "calcium-dependent phospholipase A2 activity",
  "gene": "UniProtKB:Q68DD2",
  "term_id": "GO:0047498",
  "gene_symbol": "PLA2G4F",
  "gene_name": "Cytosolic phospholipase A2 zeta"
}